{
  "gene_symbol": "SLC5A2",
  "term_id": "GO:0005886",
  "gene": "UniProtKB:P31639",
  "gene_name": "Sodium_glucose cotransporter 2",
  "term_label": "plasma membrane"
}